{
  "term_id": "UNKNOWN:0003",
  "gene_name": "Probable non-functional immunoglobulin heavy variable 3-35",
  "term_label": "Unknown cellular component",
  "gene": "UniProtKB:A0A0C4DH35",
  "gene_symbol": "IGHV3-35"
}